regulation of L-glutamine biosynthetic process [GO:0062132] (BP) Subtypes: negative regulation of L-glutamine biosynthetic process [GO:0062133], positive regulation of L-glutamine biosynthetic process [GO:0062134] References: PMID:19755423 Sources: GOC:ha Relationships: is a type of GO:0062012; is_a regulation of amino acid biosynthetic process [GO:2000282]; regulates L-glutamine biosynthetic process [GO:1901704] Definition: Any process that modulates the rate, frequency or extent of L-glutamine biosynthesis.